(1->3)-beta-D-glucan catabolic process [GO:0006076] (biological process) Sources: GOC:ai Definition: The chemical reactions and pathways resulting in the breakdown of (1->3)-beta-D-glucans. Also known as: 1,3-beta-D-glucan catabolic process, 1,3-beta-glucan breakdown, 1,3-beta-glucan catabolism, 1,3-beta-glucan degradation, beta-1,3 glucan breakdown, beta-1,3 glucan catabolic process, beta-1,3 glucan catabolism, beta-1,3 glucan degradation Relationships: is a type of (1->3)-beta-D-glucan metabolic process [GO:0006074]; is a type of beta-glucan catabolic process [GO:0051275]